nucleus disassembly [GO:1905690] (biological process) Relationships: is a type of nucleus organization [GO:0006997]; is a type of GO:1903008 Definition: The disaggregation of a nucleus into its constituent components. Sources: GOC:TermGenie, GOC:autophagy, GOC:pr, GO_REF:0000079 Also known as: cell nucleus disassembly